{
  "term_label": "membrane fusion",
  "gene_symbol": "HACE1",
  "gene": "UniProtKB:Q8IYU2",
  "gene_name": "E3 ubiquitin-protein ligase HACE1",
  "term_id": "GO:0061025"
}